{
  "gene_name": "Putative cTAGE family member 3",
  "term_id": "UNKNOWN:0001",
  "gene_symbol": "CTAGE3P",
  "gene": "UniProtKB:Q8IX95",
  "term_label": "Unknown molecular function"
}